{
  "gene": "UniProtKB:A0A494C176",
  "gene_name": "Uncharacterized protein",
  "term_label": "Unknown molecular function",
  "gene_symbol": "A0A494C176",
  "term_id": "UNKNOWN:0001"
}